{
  "term_label": "negative regulation of transcription by RNA polymerase III",
  "gene_symbol": "MAF1",
  "gene": "UniProtKB:Q9H063",
  "term_id": "GO:0016480",
  "gene_name": "Repressor of RNA polymerase III transcription MAF1 homolog"
}